{
  "gene_name": "Microfibrillar-associated protein 5",
  "term_id": "GO:0048048",
  "term_label": "embryonic eye morphogenesis",
  "gene_symbol": "MFAP5",
  "gene": "UniProtKB:Q13361"
}